{
  "term_id": "UNKNOWN:0003",
  "term_label": "Unknown cellular component",
  "gene_symbol": "TPP1",
  "gene": "UniProtKB:O14773",
  "gene_name": "Tripeptidyl-peptidase 1"
}